{
  "gene_symbol": "CGB2",
  "gene_name": "Choriogonadotropin subunit beta variant 2",
  "gene": "UniProtKB:Q6NT52",
  "term_label": "hormone activity",
  "term_id": "GO:0005179"
}